2,4-dichlorophenoxyacetate alpha-ketoglutarate dioxygenase activity [GO:0018602] (molecular function) Sources: UM-BBD_reactionID:r0274 Relationships: is_a 2-oxoglutarate-dependent dioxygenase activity [GO:0016706] Definition: Catalysis of the reaction: 2,4-dichlorophenoxyacetate + 2-oxoglutarate + oxygen = 2,4-dichlorophenol + glyoxylate + succinate + CO2.